2',3'-cyclic-nucleotide 3'-phosphodiesterase activity [GO:0004113] (molecular function) Also known as: 2',3'-cyclic nucleoside monophosphate phosphodiesterase, 2',3'-cyclic nucleotide phosphohydrolase, cyclic 2',3'-nucleotide phosphodiesterase, 2',3'-cyclic nucleotide 3'-phosphodiesterase activity, cyclic-CMP phosphodiesterase activity, 2',3'-cyclic AMP phosphodiesterase activity, 2',3'-cyclic nucleotide 3'-phosphohydrolase activity, 2':3'-CNMP-3'-ase activity, 2':3'-cyclic nucleotide 3'-phosphodiesterase activity, CNPase activity, cyclic 2',3'-nucleotide 3'-phosphodiesterase activity, nucleoside-2',3'-cyclic-phosphate 2'-nucleotidohydrolase activity Definition: Catalysis of the reaction: nucleoside 2',3'-cyclic phosphate + H2O = nucleoside 2'-phosphate. Relationships: is_a cyclic-nucleotide phosphodiesterase activity [GO:0004112] Sources: EC:3.1.4.37